chemokine (C-X-C motif) ligand 12 production [GO:0097390] (biological process) Sources: GOC:rv Relationships: is a type of GO:0032602 Also known as: CXCL12 production Definition: The appearance of chemokine (C-X-C motif) ligand 12 (CXCL12) due to biosynthesis or secretion following a cellular stimulus, resulting in an increase in its intracellular or extracellular levels.